{
  "gene": "UniProtKB:P29017",
  "gene_name": "T-cell surface glycoprotein CD1c",
  "term_label": "endogenous lipid antigen binding",
  "term_id": "GO:0030883",
  "gene_symbol": "CD1C"
}